{
  "gene_name": "Olfactory receptor 6C3",
  "gene": "UniProtKB:Q9NZP0",
  "term_id": "UNKNOWN:0002",
  "term_label": "Unknown biological process",
  "gene_symbol": "OR6C3"
}